{
  "gene_name": "B1 bradykinin receptor",
  "term_id": "GO:0004947",
  "gene": "UniProtKB:P46663",
  "term_label": "bradykinin receptor activity",
  "gene_symbol": "BDKRB1"
}